Entner-Doudoroff pathway through gluconate to D-glyceraldehyde [GO:0061680] (biological process) References: PMID:12921536 Sources: GOC:dph, MetaCyc:NPGLUCAT-PWY Relationships: is a type of non-phosphorylated glucose catabolic process [GO:0019595]; is a type of GO:0061679; is a type of glucose catabolic process to pyruvate [GO:0061718]; has part 2-dehydro-3-deoxy-D-gluconate aldolase activity [GO:0061677] Definition: The Entner-Doudoroff pathway that proceeds through a D-gluconate intermediate and yields pyruvate and D-glyceraldehyde.